{
  "gene": "UniProtKB:Q96IL0",
  "gene_symbol": "COA8",
  "gene_name": "Cytochrome c oxidase assembly factor 8",
  "term_label": "Unknown molecular function",
  "term_id": "UNKNOWN:0001"
}